endothelial tube lumen extension [GO:0097498] (biological process) References: PMID:23698350 Sources: GOC:dgh Subtypes: endothelial tube lumen extension involved in blood vessel lumen ensheathment [GO:1902355] Relationships: is a type of endothelial tube morphogenesis [GO:0061154] Definition: Any endothelial tube morphogenesis process by which the tube is increased in length.